{
  "term_id": "GO:0005634",
  "gene": "UniProtKB:P04792",
  "gene_name": "Heat shock protein beta-1",
  "gene_symbol": "HSPB1",
  "term_label": "nucleus"
}